negative regulation of translation initiation in response to endoplasmic reticulum stress [GO:0036495] (biological process) Definition: Any process that stops, prevents, or reduces the frequency, rate or extent of translation initiation as a result of endoplasmic reticulum stress. Sources: GOC:PARL, GOC:bf Also known as: negative regulation of translation initiation in response to ER stress Relationships: is a type of negative regulation of translational initiation in response to stress [GO:0032057]; is a type of regulation of translation initiation in response to endoplasmic reticulum stress [GO:0036491]; is a type of GO:1902010